{
  "term_label": "cytosol",
  "gene": "UniProtKB:P31321",
  "gene_name": "cAMP-dependent protein kinase type I-beta regulatory subunit",
  "gene_symbol": "PRKAR1B",
  "term_id": "GO:0005829"
}